{
  "term_label": "nucleus",
  "gene": "UniProtKB:Q8WYB5",
  "term_id": "GO:0005634",
  "gene_symbol": "KAT6B",
  "gene_name": "Histone acetyltransferase KAT6B"
}